{
  "term_id": "GO:0030971",
  "term_label": "receptor tyrosine kinase binding",
  "gene_name": "Copine-3",
  "gene_symbol": "CPNE3",
  "gene": "UniProtKB:O75131"
}